{
  "gene_symbol": "CLASP2",
  "term_id": "GO:0045180",
  "gene": "UniProtKB:O75122",
  "term_label": "basal cortex",
  "gene_name": "CLIP-associating protein 2"
}